glucosamine-1-phosphate N-acetyltransferase activity [GO:0019134] (molecular function) Sources: EC:2.3.1.157, RHEA:13725 Also known as: acetyl-CoA:D-glucosamine-1-phosphate N-acetyltransferase activity, acetyl-CoA:alpha-D-glucosamine-1-phosphate N-acetyltransferase activity Definition: Catalysis of the reaction: alpha-D-glucosamine 1-phosphate + acetyl-CoA = N-acetyl-alpha-D-glucosamine 1-phosphate + CoA + H+. Relationships: is a type of GO:0008080